positive regulation of blood pressure [GO:0045777] (biological process) Sources: GOC:go_curators, GOC:mtg_cardio Definition: Any process in which the force of blood traveling through the circulatory system is increased. Relationships: is a type of regulation of blood pressure [GO:0008217] Also known as: up regulation of blood pressure, up-regulation of blood pressure, upregulation of blood pressure, activation of blood pressure, stimulation of blood pressure Subtypes: positive regulation of systemic arterial blood pressure [GO:0003084], positive regulation of blood pressure by epinephrine-norepinephrine [GO:0003321]